systemic acquired resistance [GO:0009627] (BP) Definition: The salicylic acid-mediated response to a pathogen which confers broad spectrum resistance. Regulation: regulated by regulation of systemic acquired resistance [GO:0010112]; negatively regulated by negative regulation of systemic acquired resistance [GO:0010113]; negatively regulated by GO:0052003; positively regulated by positive regulation of systemic acquired resistance [GO:1901672] Sources: GOC:lr, Wikipedia:Systemic_acquired_resistance Relationships: is a type of defense response to symbiont [GO:0140546] Also known as: salicylic acid-dependent systemic resistance